positive regulation of protein tyrosine kinase activity [GO:0061098] (biological process) Relationships: is a type of positive regulation of protein kinase activity [GO:0045860]; is a type of positive regulation of peptidyl-tyrosine phosphorylation [GO:0050731]; is a type of regulation of protein tyrosine kinase activity [GO:0061097]; RO_0002213 protein tyrosine kinase activity [GO:0004713] Sources: GOC:dph, GOC:tb Definition: Any process that increases the rate, frequency, or extent of protein tyrosine kinase activity.